initiator methionyl aminopeptidase activity [GO:0004239] (molecular function) Also known as: L-methionine aminopeptidase activity, MAP, methionine aminopeptidase activity, peptidase M activity Sources: EC:3.4.11.18 Note: This term was reinstated from obsolete Definition: Catalysis of the release of N-terminal initiator methionine from peptides. Relationships: is a type of aminopeptidase activity [GO:0004177]